{
  "gene": "UniProtKB:Q96JI7",
  "term_id": "UNKNOWN:0001",
  "gene_name": "Spatacsin",
  "gene_symbol": "SPG11",
  "term_label": "Unknown molecular function"
}